{
  "term_id": "GO:0005523",
  "term_label": "tropomyosin binding",
  "gene": "UniProtKB:Q6P5Q4",
  "gene_name": "Leiomodin-2",
  "gene_symbol": "LMOD2"
}